{
  "term_id": "GO:0005814",
  "term_label": "centriole",
  "gene_name": "Centrosomal protein of 97 kDa",
  "gene_symbol": "CEP97",
  "gene": "UniProtKB:Q8IW35"
}